{
  "term_id": "UNKNOWN:0002",
  "gene_symbol": "SAPCD2",
  "gene": "UniProtKB:Q86UD0",
  "gene_name": "Suppressor APC domain-containing protein 2",
  "term_label": "Unknown biological process"
}